{
  "gene_name": "Cullin-5",
  "term_label": "ubiquitin ligase complex scaffold activity",
  "gene": "UniProtKB:Q93034",
  "gene_symbol": "CUL5",
  "term_id": "GO:0160072"
}